{
  "gene_symbol": "ACAD11",
  "term_label": "fatty acid beta-oxidation using acyl-CoA dehydrogenase",
  "gene": "UniProtKB:Q709F0",
  "term_id": "GO:0033539",
  "gene_name": "Acyl-CoA dehydrogenase family member 11"
}